structural constituent of synapse-associated extracellular matrix [GO:0150043] (molecular function) Also known as: extra-synaptic extracellular matrix structural constituent, structural constituent of extra-synaptic extracellular matrix, synapse-associated extracellular matrix structural constituent References: PMID:17189701 Sources: GOC:aruk, GOC:bc Definition: The action of a molecule that contributes to the structural integrity of the extracellular matrix of the perisynaptic space (the extracellular space adjacent to the synapse) and the synaptic cleft. Relationships: is_a extracellular matrix structural constituent [GO:0005201]; occurs in synapse-associated extracellular matrix [GO:0099535]